{
  "gene_name": "T cell receptor alpha joining 50 (Fragment)",
  "term_id": "UNKNOWN:0003",
  "gene": "UniProtKB:A0A075B6X7",
  "term_label": "Unknown cellular component",
  "gene_symbol": "TRAJ50"
}